{
  "gene_name": "Plakophilin-2",
  "gene": "UniProtKB:Q99959",
  "gene_symbol": "PKP2",
  "term_label": "nucleus",
  "term_id": "GO:0005634"
}